{
  "gene_name": "Rhox homeobox family member 1",
  "gene_symbol": "RHOXF1",
  "term_id": "GO:0005634",
  "gene": "UniProtKB:Q8NHV9",
  "term_label": "nucleus"
}